{
  "term_id": "GO:0005886",
  "term_label": "plasma membrane",
  "gene_name": "Hemojuvelin",
  "gene": "UniProtKB:Q6ZVN8",
  "gene_symbol": "HJV"
}